{
  "gene_symbol": "PPP6R2",
  "gene_name": "Serine_threonine-protein phosphatase 6 regulatory subunit 2",
  "gene": "UniProtKB:O75170",
  "term_label": "protein phosphatase regulator activity",
  "term_id": "GO:0019888"
}